{
  "gene_symbol": "FAS",
  "gene_name": "Tumor necrosis factor receptor superfamily member 6",
  "term_label": "activation-induced cell death of T cells",
  "gene": "UniProtKB:P25445",
  "term_id": "GO:0006924"
}